{
  "gene_symbol": "HLA-DMB",
  "term_label": "positive regulation of T cell activation",
  "gene": "UniProtKB:P28068",
  "gene_name": "HLA class II histocompatibility antigen, DM beta chain",
  "term_id": "GO:0050870"
}